{
  "gene": "UniProtKB:A0A087WW49",
  "gene_symbol": "LOC102724971",
  "gene_name": "Ig-like domain-containing protein (Fragment)",
  "term_id": "GO:0016064",
  "term_label": "immunoglobulin mediated immune response"
}